{
  "gene_symbol": "RTL1",
  "term_label": "placenta development",
  "gene_name": "Retrotransposon-like protein 1",
  "gene": "UniProtKB:A6NKG5",
  "term_id": "GO:0001890"
}